9+0 non-motile cilium [GO:0097731] (cellular component) Subtypes: photoreceptor cell cilium [GO:0097733] Relationships: is a type of non-motile cilium [GO:0097730] Also known as: 9+0 immotile cilium, non-motile 9+0 cilium, primary cilium References: PMID:22118931 Sources: GOC:cilia Note: This type of cilia may be present in solitary (authentic primary cilia in many cell types) or in multiple copies (e.g. in Grueneberg ganglion neurons). Definition: A non-motile cilium where the axoneme has a ring of nine outer microtubule doublets but no central microtubules (and is therefore called a 9+0 axoneme).